homoserine biosynthetic process [GO:0009090] (biological process) Relationships: is a type of GO:0009070; is a type of homoserine metabolic process [GO:0009092] Regulation: regulated by regulation of homoserine biosynthetic process [GO:1901710]; negatively regulated by negative regulation of homoserine biosynthetic process [GO:1901711]; positively regulated by positive regulation of homoserine biosynthetic process [GO:1901712] Also known as: homoserine anabolism, homoserine biosynthesis, homoserine formation, homoserine synthesis Definition: The chemical reactions and pathways resulting in the formation of homoserine, alpha-amino-gamma-hydroxybutyric acid. Sources: GOC:go_curators, ISBN:0198506732